sulfonylurea receptor binding [GO:0017098] (molecular function) Definition: Binding to a sulfonylurea receptor, a regulatory subunit of the ATP-sensitive potassium ion channel. References: PMID:11938023 Sources: GOC:ceb Also known as: sulphonylurea receptor binding, sulfonylurea receptor ligand Relationships: is a type of GO:0005102